{
  "gene": "UniProtKB:P48551",
  "gene_name": "Interferon alpha_beta receptor 2",
  "gene_symbol": "IFNAR2",
  "term_label": "plasma membrane",
  "term_id": "GO:0005886"
}